{
  "term_label": "5'-flap endonuclease activity",
  "gene": "UniProtKB:Q17RS7",
  "gene_symbol": "GEN1",
  "gene_name": "Flap endonuclease GEN homolog 1",
  "term_id": "GO:0017108"
}